orsellinate decarboxylase activity [GO:0050159] (molecular function) Relationships: is a type of carboxy-lyase activity [GO:0016831] Sources: EC:4.1.1.58, RHEA:16733 Also known as: orsellinate carboxy-lyase (orcinol-forming), orsellinate carboxy-lyase activity Definition: Catalysis of the reaction: o-orsellinate + H+ = CO2 + orcinol.